{
  "gene_name": "Ankyrin repeat domain-containing protein 20A1",
  "gene_symbol": "ANKRD20A1",
  "term_label": "Unknown biological process",
  "gene": "UniProtKB:Q5TYW2",
  "term_id": "UNKNOWN:0002"
}